seed development [GO:0048316] (biological process) Definition: The process whose specific outcome is the progression of the seed over time, from its formation to the mature structure. A seed is a propagating organ formed in the sexual reproductive cycle of gymnosperms and angiosperms, consisting of a protective coat enclosing an embryo and food reserves. Sources: GOC:jid, PO:0009010 Relationships: is a type of GO:0009791; is a type of reproductive structure development [GO:0048608]; is part of GO:0010154 Regulation: regulated by regulation of seed development [GO:0080050]